{
  "term_label": "positive regulation of action potential",
  "gene_symbol": "NPS",
  "gene_name": "Neuropeptide S",
  "term_id": "GO:0045760",
  "gene": "UniProtKB:P0C0P6"
}